{
  "term_id": "GO:0047946",
  "gene_name": "Glycine N-acyltransferase-like protein 1",
  "gene_symbol": "GLYATL1",
  "gene": "UniProtKB:Q969I3",
  "term_label": "glutamine N-acyltransferase activity"
}